tRNA 2-(methylsulfanyl)-N(6)-isopentenyladenosine(37) hydroxylase activity [GO:0045301] (MF) Also known as: 2-methylthio-cis-ribozeatin hydroxylase activity, tRNA-(2-methylthio-N-6-(cis-hydroxy)isopentenyl adenosine)-hydroxylase activity, tRNA-(2-methylthio-N-6-(cis-hydroxy)isopentenyladenosine)-hydroxylase activity, tRNA-(ms2io6A)-hydroxylase activity References: PMID:8253666 Sources: RHEA:65812 Definition: Catalysis of the reaction: 2-methylsulfanyl-N(6)-dimethylallyladenosine(37) in tRNA + acceptor-H2 + O2 = N(6)-[(2E)-4-hydroxy-3-methylbut-2-en-1-yl]-2-(methylsulfanyl)adenosine(37) in tRNA + acceptor + H2O. Relationships: is_a oxidoreductase activity, acting on paired donors, with incorporation or reduction of molecular oxygen [GO:0016705]; is a type of catalytic activity, acting on a tRNA [GO:0140101]